{
  "gene_name": "DCN1-like protein 3",
  "gene": "UniProtKB:Q8IWE4",
  "gene_symbol": "DCUN1D3",
  "term_label": "ubiquitin conjugating enzyme binding",
  "term_id": "GO:0031624"
}